intrinsic apoptotic signaling pathway in response to hydrogen peroxide [GO:0036481] (biological process) Definition: The series of molecular signals in which an intracellular signal is conveyed to trigger the apoptotic death of a cell. The pathway is induced in response to hydrogen peroxide (H2O2). Sources: GOC:PARL, GOC:bf Also known as: hydrogen peroxide-induced apoptosis, hydrogen peroxide-induced intrinsic apoptotic signaling pathway, intrinsic apoptotic signaling pathway in response to H2O2, H2O2-induced intrinsic apoptotic signaling pathway Subtypes: neuron intrinsic apoptotic signaling pathway in response to hydrogen peroxide [GO:0036482] Relationships: is_a intrinsic apoptotic signaling pathway in response to oxidative stress [GO:0008631]; is part of hydrogen peroxide-mediated programmed cell death [GO:0010421] Regulation: regulated by regulation of intrinsic apoptotic signaling pathway in response to hydrogen peroxide [GO:1903750]; negatively regulated by negative regulation of intrinsic apoptotic signaling pathway in response to hydrogen peroxide [GO:1903751]; positively regulated by GO:1903752